{
  "gene": "UniProtKB:Q8N8Y2",
  "term_label": "early endosome",
  "gene_name": "V-type proton ATPase subunit d 2",
  "term_id": "GO:0005769",
  "gene_symbol": "ATP6V0D2"
}